purine ribonucleoside catabolic process [GO:0046130] (biological process) Definition: The chemical reactions and pathways resulting in the breakdown of any purine ribonucleoside, a nucleoside in which purine base is linked to a ribose (beta-D-ribofuranose) molecule. Also known as: purine ribonucleoside breakdown, purine ribonucleoside catabolism, purine ribonucleoside degradation Subtypes: GO:0006148, adenosine catabolic process [GO:0006154], S-adenosylhomocysteine catabolic process [GO:0019510], GO:1901069, GO:1903228 Relationships: is_a purine nucleoside catabolic process [GO:0006152]; is a type of ribonucleoside catabolic process [GO:0042454]; is a type of purine ribonucleoside metabolic process [GO:0046128] Sources: GOC:ai